peptide pheromone secretion [GO:0090538] (biological process) Definition: The regulated release of a peptide pheromone from a cell. Sources: GOC:al, GOC:tb, GOC:vw Relationships: is a type of peptide pheromone export [GO:0000770]; is a type of peptide hormone secretion [GO:0030072]